cell death [GO:0008219] (biological process) References: PMID:25236395 Sources: GOC:mah, GOC:mtg_apoptosis Subtypes: programmed cell death [GO:0012501] Also known as: accidental cell death, necrosis Relationships: is a type of GO:0009987 Note: This term should not be used for direct annotation, it is currently kept in GO as a placeholder for describing cell death phenotypes in uPHENO. When information is provided on a programmed cell death mechanism, annotations should be made to the appropriate descendant of 'cell death' (such as, but not limited to, GO:0097300 'programmed necrotic cell death' or GO:0006915 'apoptotic process'). Unintentional cell death, i.e. cell death caused by injury, ageing, or cell phenotypes observed as a result of a pathological mutation in an essential gene should NOT be annotated using GO terms. Definition: Any biological process that results in permanent cessation of all vital functions of a cell. A cell should be considered dead when any one of the following molecular or morphological criteria is met: (1) the cell has lost the integrity of its plasma membrane; (2) the cell, including its nucleus, has undergone complete fragmentation into discrete bodies (frequently referred to as apoptotic bodies). The cell corpse (or its fragments) may be engulfed by an adjacent cell in vivo, but engulfment of whole cells should not be considered a strict criteria to define cell death as, under some circumstances, live engulfed cells can be released from phagosomes (see PMID:18045538).